{
  "term_id": "GO:0150007",
  "gene": "UniProtKB:Q9NZM3",
  "gene_symbol": "ITSN2",
  "term_label": "clathrin-dependent synaptic vesicle endocytosis",
  "gene_name": "Intersectin-2"
}